{
  "gene_symbol": "FXYD5",
  "term_id": "UNKNOWN:0003",
  "gene": "UniProtKB:Q96DB9",
  "gene_name": "FXYD domain-containing ion transport regulator 5",
  "term_label": "Unknown cellular component"
}